regulation of ATP-dependent activity [GO:0043462] (biological process) Sources: GOC:jl Relationships: is a type of regulation of molecular function [GO:0065009]; regulates GO:0140657 Also known as: regulation of ATPase activity, regulation of adenosinetriphosphatase activity Definition: Any process that modulates the rate of an ATP-dependent activity. Subtypes: negative regulation of ATP-dependent activity [GO:0032780], positive regulation of ATP-dependent activity [GO:0032781], regulation of ATPase-coupled calcium transmembrane transporter activity [GO:1901894], GO:1902280, regulation of P-type sodium:potassium-exchanging transporter activity [GO:1903406], regulation of potassium:proton exchanging ATPase activity [GO:1904451]